{
  "gene_name": "BolA-like protein 3",
  "term_label": "Unknown molecular function",
  "term_id": "UNKNOWN:0001",
  "gene_symbol": "BOLA3",
  "gene": "UniProtKB:Q53S33"
}